{
  "gene": "UniProtKB:Q969E3",
  "term_id": "GO:0051429",
  "gene_name": "Urocortin-3",
  "term_label": "corticotropin-releasing hormone receptor binding",
  "gene_symbol": "UCN3"
}